motile cilium assembly [GO:0044458] (biological process) Also known as: motile primary cilia assembly, motile primary cilia formation, motile primary cilium assembly, motile primary cilium formation, nodal cilium assembly, nodal cilium formation Regulation: regulated by GO:1905503; negatively regulated by negative regulation of motile cilium assembly [GO:1905504]; positively regulated by positive regulation of motile cilium assembly [GO:1905505] Subtypes: paraflagellar rod assembly [GO:0120268], sperm flagellum assembly [GO:0120316] References: PMID:19776033, PMID:21129373 Sources: GOC:TermGenie, GOC:cilia, GOC:krc, GO_REF:0000079, ZFIN:dsf Definition: The aggregation, arrangement and bonding together of a set of components to form a motile cilium. Relationships: is_a cilium assembly [GO:0060271]